{
  "term_id": "UNKNOWN:0002",
  "gene_symbol": "ZNF788P",
  "gene_name": "Putative KRAB domain-containing protein ZNF788",
  "term_label": "Unknown biological process",
  "gene": "UniProtKB:Q6ZQV5"
}